{
  "gene_name": "Putative beta-actin-like protein 3",
  "term_id": "GO:0035267",
  "gene_symbol": "POTEKP",
  "gene": "UniProtKB:Q9BYX7",
  "term_label": "NuA4 histone acetyltransferase complex"
}